{
  "term_id": "GO:0005886",
  "gene_symbol": "LLGL2",
  "term_label": "plasma membrane",
  "gene": "UniProtKB:Q6P1M3",
  "gene_name": "LLGL scribble cell polarity complex component 2"
}